hydroxylamine oxidase activity [GO:0047991] (molecular function) Definition: Catalysis of the reaction: hydroxylamine + O2 = H2O + H+ + nitrite. Sources: RHEA:19969 Also known as: hydroxylamine oxidoreductase, HAO, hydroxylamine:oxygen oxidoreductase activity Relationships: is a type of oxidoreductase activity, acting on other nitrogenous compounds as donors, oxygen as acceptor [GO:0016663]